{
  "gene": "UniProtKB:Q9UPA5",
  "gene_name": "Protein bassoon",
  "term_id": "GO:0035418",
  "term_label": "protein localization to synapse",
  "gene_symbol": "BSN"
}